{
  "gene_name": "(E2-independent) E3 ubiquitin-conjugating enzyme FATS",
  "gene_symbol": "C10orf90",
  "term_id": "GO:0005829",
  "gene": "UniProtKB:Q96M02",
  "term_label": "cytosol"
}